plant ovule development [GO:0048481] (biological process) Definition: The process whose specific outcome is the progression of the ovule over time, from its formation to the mature structure. The ovule is the structure in seed plants enclosing the female gametophyte, and is composed of the nucellus, one or two integuments, and the funiculus; it develops into the seed. Relationships: is a type of developmental process involved in reproduction [GO:0003006]; is a type of plant organ development [GO:0099402]; is part of plant-type ovary development [GO:0035670] Sources: GOC:tb